activin receptor activity, type II [GO:0016362] (molecular function) Relationships: is a type of activin receptor activity [GO:0017002] Definition: Combining with activin to initiate a change in cell activity; upon ligand binding, binds to and catalyses the phosphorylation of a type I activin receptor. References: PMID:8622651 Sources: GOC:mah Also known as: type II activin receptor activity